lobar bronchus epithelium development [GO:0060481] (biological process) Definition: The biological process whose specific outcome is the progression of a lobar bronchus epithelium from an initial condition to its mature state. This process begins with the formation of the lobar bronchus epithelium and ends with the mature structure. The lobar bronchus epithelium is the tissue made up of epithelial cells that lines the inside of the lobar bronchus. Sources: GOC:dph, GOC:mtg_lung Relationships: is a type of GO:0060428; is part of lobar bronchus development [GO:0060482]